{
  "term_id": "GO:0031410",
  "gene_name": "Trafficking kinesin-binding protein 1",
  "gene": "UniProtKB:Q9UPV9",
  "gene_symbol": "TRAK1",
  "term_label": "cytoplasmic vesicle"
}